5-formyltetrahydrofolate transport [GO:0015885] (biological process) Definition: The directed movement of 5-formyltetrahydrofolate, the formylated derivative of tetrahydrofolate, into, out of, within, or between cells, by means of some agent such as a transporter or pore. Relationships: is a type of dicarboxylic acid transport [GO:0006835]; is_a modified amino acid transport [GO:0072337] Sources: GOC:ai